{
  "gene_name": "Cytohesin-3",
  "term_label": "plasma membrane",
  "gene": "UniProtKB:O43739",
  "term_id": "GO:0005886",
  "gene_symbol": "CYTH3"
}